acquisition of desiccation tolerance in seed [GO:0048700] (BP) Sources: GOC:PO_curators, GOC:jid, GOC:ki, ISBN:9781405139830 Also known as: acquisition of desiccation tolerance Relationships: is a type of GO:0003006; is a type of acquisition of desiccation tolerance [GO:0097439]; is part of GO:0010162 Definition: The process in which a seed acquires tolerance to severe drying, before entering into a dry, either dormant or quiescent state.